{
  "gene_name": "Centrosomal protein of 162 kDa",
  "term_id": "UNKNOWN:0001",
  "gene_symbol": "CEP162",
  "term_label": "Unknown molecular function",
  "gene": "UniProtKB:Q5TB80"
}